{
  "gene_symbol": "LRRC7",
  "gene": "UniProtKB:Q96NW7",
  "term_id": "GO:0098609",
  "gene_name": "Leucine-rich repeat-containing protein 7",
  "term_label": "cell-cell adhesion"
}